adenylate cyclase regulator activity [GO:0010854] (molecular function) Subtypes: GO:0010855, adenylate cyclase activator activity [GO:0010856] Relationships: is a type of cyclase regulator activity [GO:0010851]; regulates adenylate cyclase activity [GO:0004016] Sources: GOC:dph, GOC:tb Definition: Binds to and modulates the activity of adenylate cyclase.